{
  "gene_symbol": "TMEM217",
  "term_id": "UNKNOWN:0003",
  "gene": "UniProtKB:Q8N7C4",
  "gene_name": "Transmembrane protein 217",
  "term_label": "Unknown cellular component"
}